leukemia inhibitory factor receptor binding [GO:0005146] (molecular function) Definition: Binding to an leukemia inhibitory factor receptor. Sources: GOC:ai Also known as: leukemia inhibitory factor, leukemia inhibitory factor receptor ligand Relationships: is a type of cytokine receptor binding [GO:0005126]